{
  "gene_symbol": "RAP1A",
  "term_label": "cellular response to cAMP",
  "term_id": "GO:0071320",
  "gene_name": "Ras-related protein Rap-1A",
  "gene": "UniProtKB:P62834"
}